{
  "gene": "UniProtKB:Q9BRT9",
  "term_label": "GINS complex",
  "gene_symbol": "GINS4",
  "term_id": "GO:0000811",
  "gene_name": "DNA replication complex GINS protein SLD5"
}